{
  "gene_symbol": "METTL17",
  "term_id": "UNKNOWN:0002",
  "gene_name": "Methyltransferase-like protein 17, mitochondrial",
  "term_label": "Unknown biological process",
  "gene": "UniProtKB:Q9H7H0"
}